{
  "term_label": "Unknown biological process",
  "gene_name": "Zinc finger protein 592",
  "term_id": "UNKNOWN:0002",
  "gene_symbol": "ZNF592",
  "gene": "UniProtKB:Q92610"
}